(M)-viriditoxin biosynthetic process [GO:0140783] (biological process) Definition: The chemical reactions and pathways resulting in the formation of (M)-viriditoxin, a fungal secondary metabolite with antibacterial activity. References: PMID:31045362, PMID:31304040 Also known as: viriditoxin anabolism, viriditoxin biosynthesis, viriditoxin formation, viriditoxin synthesis, (M)-viriditoxin anabolism, (M)-viriditoxin biosynthesis, (M)-viriditoxin formation, (M)-viriditoxin synthesis Relationships: is a type of polyketide biosynthetic process [GO:0030639]; is a type of GO:0043386; is a type of phenol-containing compound biosynthetic process [GO:0046189]; is_a ether biosynthetic process [GO:1901503]